ventriculo bulbo valve development [GO:0003173] (biological process) Sources: GOC:mtg_heart Definition: The progression of the ventriculo bulbo valve over time, from its formation to the mature structure. Relationships: is a type of GO:0003170